{
  "gene_symbol": "DUSP4",
  "term_id": "GO:0005737",
  "gene_name": "Dual specificity protein phosphatase 4",
  "term_label": "cytoplasm",
  "gene": "UniProtKB:Q13115"
}